{
  "term_id": "UNKNOWN:0002",
  "gene_symbol": "ABCF2",
  "gene": "UniProtKB:Q9UG63",
  "gene_name": "ATP-binding cassette sub-family F member 2",
  "term_label": "Unknown biological process"
}